positive regulation of insulin secretion involved in cellular response to glucose stimulus [GO:0035774] (biological process) Definition: Any process that increases the frequency, rate or extent of the regulated release of insulin that contributes to the response of a cell to glucose. Sources: GOC:bf, GOC:yaf Also known as: positive regulation of insulin secretion in response to glucose Relationships: is a type of GO:0032024; is a type of regulation of insulin secretion involved in cellular response to glucose stimulus [GO:0061178]; positively regulates insulin secretion involved in cellular response to glucose stimulus [GO:0035773]